fat-soluble vitamin biosynthetic process [GO:0042362] (biological process) Definition: The chemical reactions and pathways resulting in the formation of any of a diverse group of vitamins that are soluble in organic solvents and relatively insoluble in water. Sources: GOC:jl, ISBN:0198506732 Also known as: fat-soluble vitamin anabolism, fat-soluble vitamin biosynthesis, fat-soluble vitamin formation, fat-soluble vitamin synthesis Relationships: is a type of vitamin biosynthetic process [GO:0009110] Subtypes: vitamin E biosynthetic process [GO:0010189], vitamin A biosynthetic process [GO:0035238], GO:0042368, vitamin K biosynthetic process [GO:0042371]